myosin IX complex [GO:0031479] (cellular component) Definition: A myosin complex containing a class IX myosin heavy chain and associated light chains. Myosin IX is monomeric with a motor domain containing an N-terminal extension and an insert in the actin binding interface, followed by four to six IQ motifs and a tail region that contains a zinc binding motif and a domain with homology to GTPase activating proteins (GAPs) of the Rho family of G-proteins. References: PMID:29679756 Relationships: is a type of unconventional myosin complex [GO:0016461]